{
  "gene_symbol": "SFTA3",
  "term_label": "Unknown molecular function",
  "term_id": "UNKNOWN:0001",
  "gene": "UniProtKB:P0C7M3",
  "gene_name": "Surfactant-associated protein 3"
}